{
  "gene_symbol": "XCR1",
  "term_id": "GO:0019957",
  "gene_name": "Chemokine XC receptor 1",
  "gene": "UniProtKB:P46094",
  "term_label": "C-C chemokine binding"
}